{
  "term_label": "positive regulation of cell population proliferation",
  "gene_name": "Mast_stem cell growth factor receptor Kit",
  "gene_symbol": "KIT",
  "term_id": "GO:0008284",
  "gene": "UniProtKB:P10721"
}